{
  "term_id": "GO:0015825",
  "gene_name": "Neutral amino acid transporter A",
  "gene": "UniProtKB:P43007",
  "gene_symbol": "SLC1A4",
  "term_label": "L-serine transport"
}